positive regulation of mesodermal to mesenchymal transition involved in gastrulation [GO:0060808] (biological process) Relationships: is a type of positive regulation of epithelial to mesenchymal transition [GO:0010718]; is a type of regulation of anatomical structure morphogenesis [GO:0022603]; positively regulates mesodermal to mesenchymal transition involved in gastrulation [GO:0060809] Definition: Any process that increases the rate, frequency, or extent of epithelial to mesenchymal transition. Epithelial to mesenchymal transition where a mesodermal cell loses apical/basolateral polarity, severs intercellular adhesive junctions, degrades basement membrane components and becomes a migratory mesenchymal cell as part of the process of gastrulation. Sources: GOC:dph, GOC:sdb_2009, GOC:tb